formate oxidation [GO:0015944] (biological process) Also known as: formic acid oxidation Definition: The chemical reactions and pathways by which formate is converted to CO2. Sources: MetaCyc:PWY-1881 Relationships: is a type of formate metabolic process [GO:0015942]